nuclear ribonucleoprotein granule [GO:0140168] (cellular component) Subtypes: Cajal body [GO:0015030], nuclear speck [GO:0016607], histone locus body [GO:0035363], paraspeckles [GO:0042382], nuclear stress granule [GO:0097165] Relationships: is a type of nuclear body [GO:0016604]; is a type of ribonucleoprotein granule [GO:0035770] Definition: A ribonucleoprotein granule located in the nucleus. References: PMID:32475683, PMID:35355287, PMID:37890457 Also known as: nuclear RNP granule, nuclear RNA granule